sexual macrocyst formation [GO:0140084] (biological process) Definition: The fusion of haploid amoebae cells with matching mating types to form a larger cell, which ingests additional amoebae and forms a cellulose wall. The resulting macrocyst undergoes recombination and meiosis followed by release of haploid amoebae. An example of this process can be found in Dictyostelium discoideum. References: PMID:16592095, PMID:20089169 Also known as: macrocyst formation, sexual fusion Relationships: is a type of reproductive process in single-celled organism [GO:0022413]